negative regulation of vernalization response [GO:0010221] (biological process) Also known as: down regulation of vernalization response, down-regulation of vernalization response, downregulation of vernalization response, inhibition of vernalization response Definition: Any process that stops, prevents or reduces the vernalization response, by which induction of flowering is normally caused by extended exposure to cold temperatures. Relationships: is a type of regulation of vernalization response [GO:0010219]; is a type of negative regulation of response to stimulus [GO:0048585]; negatively regulates vernalization response [GO:0010048] Sources: GOC:sm